{
  "term_id": "GO:0019814",
  "gene_symbol": "IGLV2-11",
  "gene": "UniProtKB:P01706",
  "gene_name": "Immunoglobulin lambda variable 2-11",
  "term_label": "immunoglobulin complex"
}